{
  "term_id": "GO:0070531",
  "term_label": "BRCA1-A complex",
  "gene_symbol": "UIMC1",
  "gene": "UniProtKB:Q96RL1",
  "gene_name": "BRCA1-A complex subunit RAP80"
}